{
  "gene": "UniProtKB:Q86TL2",
  "term_id": "GO:0016020",
  "term_label": "membrane",
  "gene_symbol": "STIMATE",
  "gene_name": "Store-operated calcium entry regulator STIMATE"
}